{
  "gene_name": "Protein SCO2 homolog, mitochondrial",
  "term_label": "Unknown molecular function",
  "gene_symbol": "SCO2",
  "term_id": "UNKNOWN:0001",
  "gene": "UniProtKB:O43819"
}